thyrotropin-releasing hormone activity [GO:0008437] (molecular function) Definition: The action characteristic of thyrotropin-releasing hormone (TRH), a hormone released by the mammalian hypothalamus into the hypophyseal-portal circulation in response to neural and/or chemical stimuli. Upon receptor binding, TRH increases the secretion of thyroid-stimulating hormone by the anterior pituitary. Sources: ISBN:0198506732 Also known as: TRH activity, thyrotropin releasing hormone activity Relationships: is a type of GO:0005179